{
  "term_id": "GO:0019005",
  "term_label": "SCF ubiquitin ligase complex",
  "gene_symbol": "FBXO48",
  "gene": "UniProtKB:Q5FWF7",
  "gene_name": "F-box only protein 48"
}